{
  "term_label": "structural molecule activity",
  "term_id": "GO:0005198",
  "gene": "UniProtKB:Q9NQW1",
  "gene_name": "Protein transport protein Sec31B",
  "gene_symbol": "SEC31B"
}